plastid thylakoid lumen [GO:0031978] (cellular component) Subtypes: chloroplast thylakoid lumen [GO:0009543], cyanelle thylakoid lumen [GO:0033114] Sources: GOC:mah Relationships: is a type of thylakoid lumen [GO:0031977]; is part of GO:0031976 Definition: The volume enclosed by a plastid thylakoid membrane.